negative regulation of synapse structural plasticity [GO:0051826] (biological process) Definition: Any process that stops, prevents, or reduces the frequency, rate or extent of synapse structural plasticity. Sources: GOC:ai Also known as: down regulation of synapse structural plasticity, down-regulation of synapse structural plasticity, downregulation of synapse structural plasticity, inhibition of synapse structural plasticity Relationships: is a type of negative regulation of cellular component organization [GO:0051129]; is a type of regulation of synapse structural plasticity [GO:0051823]